{
  "term_id": "GO:0006954",
  "term_label": "inflammatory response",
  "gene_symbol": "GPR32",
  "gene_name": "Probable G-protein coupled receptor 32",
  "gene": "UniProtKB:O75388"
}